{
  "gene_symbol": "ZNF558",
  "term_id": "GO:0006357",
  "gene_name": "Zinc finger protein 558",
  "gene": "UniProtKB:Q96NG5",
  "term_label": "regulation of transcription by RNA polymerase II"
}